{
  "gene_symbol": "SLC31A1",
  "term_id": "GO:0005886",
  "gene": "UniProtKB:O15431",
  "term_label": "plasma membrane",
  "gene_name": "High affinity copper uptake protein 1"
}